{
  "term_label": "Unknown molecular function",
  "term_id": "UNKNOWN:0001",
  "gene_symbol": "UPK3BL2",
  "gene_name": "Uroplakin-3b-like protein 2",
  "gene": "UniProtKB:E5RIL1"
}